{
  "gene_name": "WW domain-containing transcription regulator protein 1",
  "gene": "UniProtKB:Q9GZV5",
  "term_id": "GO:0060828",
  "gene_symbol": "WWTR1",
  "term_label": "regulation of canonical Wnt signaling pathway"
}